{
  "gene_name": "L-xylulose reductase",
  "term_label": "Unknown cellular component",
  "gene_symbol": "DCXR",
  "term_id": "UNKNOWN:0003",
  "gene": "UniProtKB:Q7Z4W1"
}